{
  "gene_symbol": "FAM174A",
  "term_id": "UNKNOWN:0002",
  "term_label": "Unknown biological process",
  "gene": "UniProtKB:Q8TBP5",
  "gene_name": "Membrane protein FAM174A"
}